body morphogenesis [GO:0010171] (biological process) Relationships: is a type of anatomical structure morphogenesis [GO:0009653] Definition: The process in which the anatomical structures of the soma are generated and organized. Subtypes: embryonic body morphogenesis [GO:0010172], post-embryonic body morphogenesis [GO:0040032] Sources: GOC:ems, ISBN:0140512888